regulation of calcium-dependent activation of synaptic vesicle fusion [GO:0150037] (biological process) Definition: Any process that modulates the frequency, rate or extent of calcium-dependent activation of synaptic vesicle fusion. Relationships: is a type of regulation of synaptic vesicle fusion to presynaptic active zone membrane [GO:0031630]; regulates calcium-dependent activation of synaptic vesicle fusion [GO:0099502] References: PMID:27052163 Sources: GOC:aruk, GOC:bc